regulation of metaphase/anaphase transition of meiotic cell cycle [GO:1902102] (biological process) Definition: Any process that modulates the frequency, rate or extent of metaphase/anaphase transition of meiotic cell cycle. Also known as: regulation of meiotic metaphase/anaphase transition Subtypes: negative regulation of metaphase/anaphase transition of meiotic cell cycle [GO:1902103], positive regulation of metaphase/anaphase transition of meiotic cell cycle [GO:1902104], GO:1905186, regulation of metaphase/anaphase transition of meiosis II [GO:1905189], GO:1905325 Relationships: is a type of regulation of meiotic cell cycle phase transition [GO:1901993]; is_a regulation of metaphase/anaphase transition of cell cycle [GO:1902099]; is a type of regulation of meiotic chromosome separation [GO:1905132]; regulates metaphase/anaphase transition of meiotic cell cycle [GO:0044785] Sources: GOC:TermGenie, GOC:mtg_cell_cycle